{
  "gene_name": "Stonin-1",
  "gene_symbol": "STON1",
  "term_id": "GO:0048488",
  "term_label": "synaptic vesicle endocytosis",
  "gene": "UniProtKB:Q9Y6Q2"
}